3''-deamino-3''-oxonicotianamine reductase activity [GO:0033707] (molecular function) Also known as: 2'-deoxymugineic acid:NAD(P)+ 3''-oxidoreductase activity Definition: Catalysis of the reaction: 2'-deoxymugineic acid + NAD(P)+ = 3''-deamino-3''-oxonicotianamine + NAD(P)H + H+. Sources: EC:1.1.1.285 Relationships: is a type of oxidoreductase activity, acting on the CH-OH group of donors, NAD or NADP as acceptor [GO:0016616]